{
  "gene_name": "Zinc finger protein 418",
  "term_label": "RNA polymerase II cis-regulatory region sequence-specific DNA binding",
  "gene": "UniProtKB:Q8TF45",
  "gene_symbol": "ZNF418",
  "term_id": "GO:0000978"
}